meiosis I [GO:0007127] (biological process) Regulation: regulated by GO:0060631; positively regulated by positive regulation of meiosis I [GO:0060903]; negatively regulated by negative regulation of meiosis I [GO:0110029] Subtypes: achiasmate meiosis I [GO:0000705], male meiosis I [GO:0007141], GO:0007144 Also known as: meiosis I nuclear division Relationships: is a type of meiosis I cell cycle process [GO:0061982]; is a type of meiotic nuclear division [GO:0140013]; ends during meiotic telophase I [GO:0007134] Definition: The first meiotic nuclear division in which homologous chromosomes are paired and segregated from each other, producing two haploid daughter nuclei. References: PMID:9334324 Sources: GOC:dph, GOC:jl, GOC:mtg_cell_cycle